{
  "gene_name": "Ephrin type-B receptor 4",
  "term_label": "plasma membrane",
  "gene": "UniProtKB:P54760",
  "term_id": "GO:0005886",
  "gene_symbol": "EPHB4"
}